{
  "gene": "UniProtKB:Q32NB8",
  "term_id": "GO:0008444",
  "term_label": "CDP-diacylglycerol-glycerol-3-phosphate 3-phosphatidyltransferase activity",
  "gene_name": "CDP-diacylglycerol--glycerol-3-phosphate 3-phosphatidyltransferase, mitochondrial",
  "gene_symbol": "PGS1"
}